FAT10 ligase activity [GO:0061661] (molecular function) Sources: GOC:dph Definition: Catalysis of the transfer of FAT10 to a substrate protein via the reaction X-FAT10 + S = X + S-FAT10, where X is either an E2 or E3 enzyme, the X-FAT10 linkage is a thioester bond, and the S-FAT10 linkage is an isopeptide bond between the C-terminal glycine of FAT10 and the epsilon-amino group of lysine residues in the substrate. Relationships: is a type of FAT10 transferase activity [GO:0019775]; is a type of ubiquitin-like protein ligase activity [GO:0061659] Also known as: E3